{
  "gene_name": "Calcium-activated potassium channel subunit beta-3",
  "term_id": "GO:0005513",
  "term_label": "detection of calcium ion",
  "gene": "UniProtKB:Q9NPA1",
  "gene_symbol": "KCNMB3"
}